{
  "gene_symbol": "EEF2",
  "term_id": "GO:0003746",
  "gene_name": "Elongation factor 2",
  "gene": "UniProtKB:P13639",
  "term_label": "translation elongation factor activity"
}